{
  "gene_symbol": "UBXN2A",
  "term_label": "ubiquitin binding",
  "gene_name": "UBX domain-containing protein 2A",
  "term_id": "GO:0043130",
  "gene": "UniProtKB:P68543"
}